{
  "gene_symbol": "ESRRA",
  "gene_name": "Steroid hormone receptor ERR1",
  "term_id": "GO:0004879",
  "term_label": "nuclear receptor activity",
  "gene": "UniProtKB:P11474"
}